{
  "term_label": "cytoskeleton organization",
  "gene_name": "Striatin-interacting protein 2",
  "gene": "UniProtKB:Q9ULQ0",
  "gene_symbol": "STRIP2",
  "term_id": "GO:0007010"
}